pons maturation [GO:0021586] (biological process) Sources: GOC:cls, GOC:dgh, GOC:dph, GOC:jid, GO_REF:0000021 Relationships: is a type of GO:0071695; is part of pons development [GO:0021548]; is part of hindbrain maturation [GO:0021578] Definition: A developmental process, independent of morphogenetic (shape) change, that is required for the pons to attain its fully functional state. The pons lies above the medulla and next to the cerebellum. The pons conveys information about movement from the cerebral hemisphere to the cerebellum.